{
  "gene_symbol": "SLC22A7",
  "gene": "UniProtKB:Q9Y694",
  "gene_name": "Solute carrier family 22 member 7",
  "term_id": "UNKNOWN:0002",
  "term_label": "Unknown biological process"
}